yolk plasma [GO:0060418] (cellular component) Relationships: is a type of GO:0110165; is part of yolk [GO:0060417] Definition: Discrete structures that partition the water-soluble portion of the yolk of oocytes and ova, which may or may not be membrane enclosed. References: PMID:18046696 Sources: GOC:dph, GOC:tb